{
  "gene": "UniProtKB:Q9UKW6",
  "term_id": "GO:0006357",
  "gene_name": "ETS-related transcription factor Elf-5",
  "term_label": "regulation of transcription by RNA polymerase II",
  "gene_symbol": "ELF5"
}